{
  "gene_name": "PR domain zinc finger protein 4",
  "gene": "UniProtKB:Q9UKN5",
  "term_id": "GO:0010468",
  "gene_symbol": "PRDM4",
  "term_label": "regulation of gene expression"
}